deoxycytidine catabolic process [GO:0006217] (biological process) Sources: GOC:go_curators Also known as: deoxycytidine breakdown, deoxycytidine catabolism, deoxycytidine degradation Relationships: is_a deoxycytidine metabolic process [GO:0046092]; is a type of pyrimidine deoxyribonucleoside catabolic process [GO:0046127] Definition: The chemical reactions and pathways resulting in the breakdown of deoxycytidine, 2-deoxyribosylcytosine, one of the four major nucleosides of DNA.